{
  "term_label": "cholesterol binding",
  "gene": "UniProtKB:O94905",
  "term_id": "GO:0015485",
  "gene_symbol": "ERLIN2",
  "gene_name": "Erlin-2"
}